negative regulation of protein localization to nucleus [GO:1900181] (BP) Relationships: is a type of regulation of protein localization to nucleus [GO:1900180]; is a type of negative regulation of protein localization [GO:1903828]; negatively regulates protein localization to nucleus [GO:0034504] Also known as: down regulation of protein localisation to nucleus, down regulation of protein localization in cell nucleus, down regulation of protein localization in nucleus, down regulation of protein localization to nucleus, down-regulation of protein localisation to nucleus, down-regulation of protein localization in cell nucleus, down-regulation of protein localization in nucleus, down-regulation of protein localization to nucleus, downregulation of protein localisation to nucleus, downregulation of protein localization in cell nucleus, downregulation of protein localization in nucleus, downregulation of protein localization to nucleus, negative regulation of protein localisation to nucleus, negative regulation of protein localization in cell nucleus, negative regulation of protein localization in nucleus, inhibition of protein localisation to nucleus, inhibition of protein localization in cell nucleus, inhibition of protein localization in nucleus, inhibition of protein localization to nucleus Subtypes: negative regulation of protein import into nucleus [GO:0042308], negative regulation of protein localization to nucleolus [GO:1904750], negative regulation of protein localization to Cajal body [GO:1904870] Definition: Any process that stops, prevents or reduces the frequency, rate or extent of protein localization to nucleus. Sources: GOC:TermGenie